{
  "gene": "UniProtKB:Q92966",
  "term_id": "GO:0001046",
  "term_label": "core promoter sequence-specific DNA binding",
  "gene_symbol": "SNAPC3",
  "gene_name": "snRNA-activating protein complex subunit 3"
}